regulation of interleukin-32 production [GO:0150189] (biological process) Also known as: regulation of interleukin-32 biosynthetic process, regulation of interleukin-32 secretion Relationships: is a type of GO:0001817; regulates interleukin-32 production [GO:0072637] References: PMID:23729669 Sources: GOC:aruk Definition: Any process that modulates the frequency, rate or extent of interleukin-32 production. Subtypes: negative regulation of interleukin-32 production [GO:0150190], positive regulation of interleukin-32 production [GO:0150191]